nuclear axial expansion [GO:0035191] (biological process) Relationships: is_a syncytial nuclear migration [GO:0035190] References: PMID:8314839 Definition: The stepwise asymmetric spreading out of nuclei internally along the anterior-posterior axis of the developing insect embryo during mitotic cycles 4 to 6. This movement leads to the distribution of nuclei in a hollow ellipsoid underlying the cortex. Also known as: nuclear distribution along anterior-posterior axis, nucleus distribution along anterior-posterior axis